metanephric capsule development [GO:0072213] (biological process) Sources: GOC:mtg_kidney_jan10 Definition: The process whose specific outcome is the progression of the metanephric capsule over time, from its formation to the mature structure. The metanephric capsule is the tough fibrous layer surrounding the metanephros, covered in a thick layer of perinephric adipose tissue. It provides some protection from trauma and damage. Relationships: is a type of renal capsule development [GO:0072127]; is part of metanephros development [GO:0001656]